{
  "gene_symbol": "HDAC9",
  "term_id": "GO:0040029",
  "gene": "UniProtKB:Q9UKV0",
  "term_label": "epigenetic regulation of gene expression",
  "gene_name": "Histone deacetylase 9"
}